{
  "term_id": "GO:0030424",
  "gene": "UniProtKB:Q6PCB8",
  "term_label": "axon",
  "gene_symbol": "EMB",
  "gene_name": "Embigin"
}